{
  "gene_symbol": "APOO",
  "gene": "UniProtKB:Q9BUR5",
  "term_id": "GO:0061617",
  "gene_name": "MICOS complex subunit MIC26",
  "term_label": "MICOS complex"
}